{
  "gene_symbol": "SLC39A2",
  "gene_name": "Zinc transporter ZIP2",
  "term_label": "plasma membrane",
  "gene": "UniProtKB:Q9NP94",
  "term_id": "GO:0005886"
}